{
  "gene": "UniProtKB:Q9UI38",
  "term_label": "endoplasmic reticulum",
  "gene_symbol": "PRSS50",
  "gene_name": "Probable threonine protease PRSS50",
  "term_id": "GO:0005783"
}